{
  "term_id": "GO:0045197",
  "gene_symbol": "DLG2",
  "term_label": "establishment or maintenance of epithelial cell apical/basal polarity",
  "gene_name": "Disks large homolog 2",
  "gene": "UniProtKB:Q15700"
}